{
  "term_id": "GO:0000139",
  "gene_name": "Beta-1,3-galactosyltransferase 9",
  "term_label": "Golgi membrane",
  "gene": "UniProtKB:A8MXE2",
  "gene_symbol": "B3GALT9"
}